negative regulation of motor neuron axon guidance [GO:1905813] (biological process) Relationships: is a type of negative regulation of axon guidance [GO:1902668]; is a type of GO:1905812; negatively regulates GO:0008045 Also known as: down regulation of motoneuron axon guidance, down regulation of motor axon guidance, down regulation of motor axon pathfinding, down regulation of motor neuron axon guidance, down-regulation of motoneuron axon guidance, down-regulation of motor axon guidance, down-regulation of motor axon pathfinding, down-regulation of motor neuron axon guidance, downregulation of motoneuron axon guidance, downregulation of motor axon guidance, downregulation of motor axon pathfinding, downregulation of motor neuron axon guidance, negative regulation of motoneuron axon guidance, negative regulation of motor axon guidance, negative regulation of motor axon pathfinding, inhibition of motoneuron axon guidance, inhibition of motor axon guidance, inhibition of motor axon pathfinding, inhibition of motor neuron axon guidance References: PMID:18434533 Sources: GOC:TermGenie, GO_REF:0000058 Definition: Any process that stops, prevents or reduces the frequency, rate or extent of motor neuron axon guidance.